{
  "term_label": "heterophilic cell-cell adhesion",
  "term_id": "GO:0007157",
  "gene": "UniProtKB:Q14162",
  "gene_symbol": "SCARF1",
  "gene_name": "Scavenger receptor class F member 1"
}